chimeric sorocarp development [GO:0099134] (biological process) Relationships: is_a sorocarp development [GO:0030587]; is a type of GO:0099136 References: PMID:18272966 Subtypes: GO:0099138 Definition: Development of a sorocarp formed by aggregation of cells with different genotypes.